4-hydroxy-2-ketopimelate aldolase activity [GO:0043863] (molecular function) Definition: Catalysis of the reaction: 4-hydroxy-2-ketopimelate = succinate semialdehyde + pyruvate. Sources: MetaCyc:4-HYDROXY-2-KETOPIMELATE-LYSIS-RXN Also known as: 2,4-dihydroxyhept-2-ene-1,7-dioic acid aldolase activity, HHED aldolase activity, HpaI, HpcH Relationships: is a type of aldehyde-lyase activity [GO:0016832]